{
  "term_label": "methionine adenosyltransferase activity",
  "gene_symbol": "MAT1A",
  "gene": "UniProtKB:Q00266",
  "term_id": "GO:0004478",
  "gene_name": "S-adenosylmethionine synthase isoform type-1"
}